{
  "term_label": "Mon1-Ccz1 complex",
  "gene": "UniProtKB:P86791",
  "gene_name": "Vacuolar fusion protein CCZ1 homolog",
  "term_id": "GO:0035658",
  "gene_symbol": "CCZ1"
}